trans-synaptic signaling by carbon monoxide [GO:0099549] (biological process) Sources: GOC:dos Subtypes: GO:0099556 Definition: Cell-cell signaling between presynapse and postsynapse mediated by carbon monoxide. Relationships: is a type of GO:0099543